{
  "term_id": "GO:0007286",
  "gene_name": "Testis-specific serine_threonine-protein kinase 3",
  "gene": "UniProtKB:Q96PN8",
  "term_label": "spermatid development",
  "gene_symbol": "TSSK3"
}